negative regulation of retinal cell programmed cell death [GO:0046671] (BP) Sources: GOC:ai, GOC:tb Definition: Any process that stops, prevents, or reduces the frequency, rate or extent of programmed cell death that occurs in the retina. Relationships: is a type of negative regulation of programmed cell death [GO:0043069]; is a type of regulation of retinal cell programmed cell death [GO:0046668]; is a type of negative regulation of developmental process [GO:0051093]; negatively regulates retinal cell programmed cell death [GO:0046666] Subtypes: GO:0046673 Also known as: down regulation of retinal programmed cell death, down-regulation of retinal programmed cell death, downregulation of retinal programmed cell death, negative regulation of retinal programmed cell death, inhibition of retinal programmed cell death